tRNA 4-demethylwyosine alpha-amino-alpha-carboxypropyltransferase activity [GO:0102522] (molecular function) Relationships: is a type of GO:0016765; is a type of catalytic activity, acting on a tRNA [GO:0140101] Definition: Catalysis of the reaction: S-adenosyl-L-methionine + 4-demethylwyosine37 in tRNAPhe = 5'-S-methyl-5'-thioadenosine + H+ + 7-[(3S)-3-amino-3-carboxypropyl]-4-demethylwyosine37 in tRNAPhe. Sources: EC:2.5.1.114, GOC:pz